{
  "gene_name": "V-type proton ATPase subunit C 1",
  "term_label": "Unknown biological process",
  "gene_symbol": "ATP6V1C1",
  "term_id": "UNKNOWN:0002",
  "gene": "UniProtKB:P21283"
}